{
  "gene_name": "Mitochondrial import receptor subunit TOM20 homolog",
  "term_label": "tRNA import into mitochondrion",
  "term_id": "GO:0016031",
  "gene_symbol": "TOMM20",
  "gene": "UniProtKB:Q15388"
}